{
  "gene_symbol": "EPB41L5",
  "term_id": "GO:0005856",
  "term_label": "cytoskeleton",
  "gene_name": "Band 4.1-like protein 5",
  "gene": "UniProtKB:Q9HCM4"
}